{
  "term_label": "cytoplasm",
  "gene_symbol": "MYL10",
  "gene": "UniProtKB:Q9BUA6",
  "term_id": "GO:0005737",
  "gene_name": "Myosin regulatory light chain 10"
}